camphor 5-monooxygenase activity [GO:0018683] (molecular function) Also known as: camphor 5-exo-methylene hydroxylase activity, (+)-camphor,reduced putidaredoxin:oxygen oxidoreductase (5-hydroxylating), 2-bornanone 5-exo-hydroxylase activity, D-camphor-exo-hydroxylase activity, bornanone 5-exo-hydroxylase activity, camphor 5-exo-hydroxylase activity, camphor 5-exohydroxylase activity, camphor hydroxylase activity, camphor methylene hydroxylase activity, cytochrome p450-cam activity, d-camphor monooxygenase activity, methylene hydroxylase activity, methylene monooxygenase activity Sources: EC:1.14.15.1 Relationships: is a type of oxidoreductase activity, acting on paired donors, with incorporation or reduction of molecular oxygen, reduced iron-sulfur protein as one donor, and incorporation of one atom of oxygen [GO:0016713] Definition: Catalysis of the reaction: (+)-camphor + putidaredoxin + O2 = (+)-exo-5-hydroxycamphor + oxidized putidaredoxin + H2O.